{
  "term_id": "GO:0097536",
  "gene": "UniProtKB:O43918",
  "term_label": "thymus epithelium morphogenesis",
  "gene_name": "Autoimmune regulator",
  "gene_symbol": "AIRE"
}